{
  "term_label": "cytoplasm",
  "gene_symbol": "TREX2",
  "gene_name": "Three prime repair exonuclease 2",
  "gene": "UniProtKB:Q9BQ50",
  "term_id": "GO:0005737"
}